{
  "term_label": "deoxyhypusine monooxygenase activity",
  "gene_name": "Deoxyhypusine hydroxylase",
  "gene": "UniProtKB:Q9BU89",
  "term_id": "GO:0019135",
  "gene_symbol": "DOHH"
}